neutral L-amino acid secondary active transmembrane transporter activity [GO:0005294] (molecular function) Definition: Enables the transfer of a neutral L-amino acid from one side of a membrane to the other, up its concentration gradient. The transporter binds the solute and undergoes a series of conformational changes. Transport works equally well in either direction and is driven by a chemiosmotic source of energy. Secondary active transporters include symporters and antiporters. Also known as: neutral L-amino acid porter activity Sources: GOC:mtg_transport Relationships: is a type of GO:0015175; is a type of secondary active transmembrane transporter activity [GO:0015291] Subtypes: L-methionine secondary active transmembrane transporter activity [GO:0000102]